{
  "term_id": "GO:0035556",
  "term_label": "intracellular signal transduction",
  "gene_name": "Hormonally up-regulated neu tumor-associated kinase",
  "gene_symbol": "HUNK",
  "gene": "UniProtKB:P57058"
}